regulation of chemokine (C-X-C motif) ligand 1 production [GO:2000338] (biological process) Relationships: is a type of regulation of chemokine production [GO:0032642]; regulates GO:0072566 Subtypes: negative regulation of chemokine (C-X-C motif) ligand 1 production [GO:2000339], positive regulation of chemokine (C-X-C motif) ligand 1 production [GO:2000340] Also known as: regulation of CXCL1 production, regulation of KC production, regulation of SCYB1 production, regulation of keratinocyte derived chemokine production Definition: Any process that modulates the frequency, rate or extent of chemokine (C-X-C motif) ligand 1 production. Sources: GOC:BHF, GOC:mah